{
  "gene": "UniProtKB:Q9H628",
  "term_label": "Unknown molecular function",
  "gene_name": "Ras-related and estrogen-regulated growth inhibitor-like protein",
  "gene_symbol": "RERGL",
  "term_id": "UNKNOWN:0001"
}